{
  "term_id": "GO:0002181",
  "term_label": "cytoplasmic translation",
  "gene_name": "Large ribosomal subunit protein eL6",
  "gene": "UniProtKB:Q02878",
  "gene_symbol": "RPL6"
}